{
  "gene_symbol": "IGHV1-46",
  "gene_name": "Immunoglobulin heavy variable 1-46",
  "term_id": "GO:0016064",
  "term_label": "immunoglobulin mediated immune response",
  "gene": "UniProtKB:P01743"
}